L-gulono-1,4-lactone dehydrogenase activity [GO:0080049] (MF) Relationships: is a type of GO:0016632 References: PMID:18190525, PMID:30112455 Sources: RHEA:47248 Definition: Catalysis of the reaction: L-gulono-1,4-lactone + 2 ferricytochrome c = L-ascorbate + 2 ferrocytochrome c.